positive regulation of monocyte aggregation [GO:1900625] (biological process) Also known as: activation of mononuclear phagocyte aggregation, positive regulation of mononuclear phagocyte aggregation, up regulation of monocyte aggregation, up regulation of mononuclear phagocyte aggregation, up-regulation of monocyte aggregation, up-regulation of mononuclear phagocyte aggregation, upregulation of monocyte aggregation, upregulation of mononuclear phagocyte aggregation, activation of monocyte aggregation Definition: Any process that activates or increases the frequency, rate or extent of monocyte aggregation. Relationships: is a type of regulation of monocyte aggregation [GO:1900623]; is a type of positive regulation of leukocyte cell-cell adhesion [GO:1903039]; positively regulates GO:0070487 Sources: GOC:BHF, GOC:TermGenie